{
  "gene": "UniProtKB:Q8N8U2",
  "term_id": "GO:0005634",
  "term_label": "nucleus",
  "gene_name": "Chromodomain Y-like protein 2",
  "gene_symbol": "CDYL2"
}